{
  "gene": "UniProtKB:A0A0J9YW22",
  "gene_symbol": "IGHD3-9",
  "term_id": "UNKNOWN:0001",
  "term_label": "Unknown molecular function",
  "gene_name": "Immunoglobulin heavy diversity 3-9 (Fragment)"
}